{
  "gene_name": "Carbohydrate sulfotransferase 3",
  "term_id": "GO:0008459",
  "gene": "UniProtKB:Q7LGC8",
  "gene_symbol": "CHST3",
  "term_label": "chondroitin 6-sulfotransferase activity"
}